{
  "gene_symbol": "IGFBP5",
  "term_label": "fibronectin binding",
  "gene": "UniProtKB:P24593",
  "gene_name": "Insulin-like growth factor-binding protein 5",
  "term_id": "GO:0001968"
}